aromatic amino acid transport [GO:0015801] (biological process) Definition: The directed movement of aromatic amino acids, amino acids with aromatic ring, into, out of or within a cell, or between cells, by means of some agent such as a transporter or pore. Sources: GOC:ai Subtypes: GO:0015827, GO:0015828, histamine secretion, neurotransmission [GO:0061538], L-histidine transmembrane transport [GO:0089709], GO:0140925, GO:1902024 Relationships: is a type of carboxylic acid transport [GO:0046942]; is a type of GO:0071705